{
  "term_label": "Unknown biological process",
  "gene_symbol": "PDCD6",
  "gene_name": "Programmed cell death protein 6",
  "gene": "UniProtKB:O75340",
  "term_id": "UNKNOWN:0002"
}